N-terminal peptidyl-serine trimethylation [GO:0035573] (biological process) Relationships: is a type of N-terminal peptidyl-serine methylation [GO:0035570] Definition: The trimethylation of the N-terminal serine of proteins to form the derivative N,N,N-trimethylserine. References: PMID:20668449